chloroplast RNA processing [GO:0031425] (biological process) Subtypes: chloroplast mRNA processing [GO:0010239] Definition: The conversion of a primary RNA molecule transcribed from a chloroplast genome into one or more mature RNA molecules. Relationships: is a type of RNA processing [GO:0006396] Sources: GOC:mah